negative regulation of blood coagulation, common pathway [GO:2000261] (biological process) Relationships: is a type of negative regulation of blood coagulation [GO:0030195]; is a type of negative regulation of protein activation cascade [GO:2000258]; is a type of GO:2000260; negatively regulates GO:0072377 Definition: Any process that stops, prevents or reduces the frequency, rate or extent of blood coagulation, common pathway. Sources: GOC:mah